{
  "term_id": "GO:0031463",
  "gene_symbol": "KLHL9",
  "term_label": "Cul3-RING ubiquitin ligase complex",
  "gene_name": "Kelch-like protein 9",
  "gene": "UniProtKB:Q9P2J3"
}